{
  "gene_name": "Kinesin-like protein KIFC3",
  "gene": "UniProtKB:Q9BVG8",
  "term_id": "GO:0008017",
  "term_label": "microtubule binding",
  "gene_symbol": "KIFC3"
}